{
  "gene_name": "Putative uncharacterized protein ANP32CP",
  "gene": "UniProtKB:O43423",
  "term_id": "GO:0005634",
  "gene_symbol": "ANP32CP",
  "term_label": "nucleus"
}